cellular response to testosterone stimulus [GO:0071394] (biological process) Regulation: regulated by regulation of cellular response to testosterone stimulus [GO:2000654]; negatively regulated by negative regulation of cellular response to testosterone stimulus [GO:2000655] Sources: GOC:mah Definition: Any process that results in a change in state or activity of a cell (in terms of movement, secretion, enzyme production, gene expression, etc.) as a result of a testosterone stimulus. Relationships: is a type of response to testosterone [GO:0033574]; is a type of cellular response to lipid [GO:0071396]; is a type of cellular response to ketone [GO:1901655]